{
  "gene_symbol": "F8",
  "gene_name": "Coagulation factor VIII",
  "term_id": "GO:0005615",
  "gene": "UniProtKB:P00451",
  "term_label": "extracellular space"
}